{
  "term_id": "GO:0003886",
  "gene_symbol": "DNMT1",
  "gene_name": "DNA (cytosine-5)-methyltransferase 1",
  "term_label": "DNA (cytosine-5-)-methyltransferase activity",
  "gene": "UniProtKB:P26358"
}